{
  "gene_symbol": "MASP2",
  "term_id": "GO:0001867",
  "gene": "UniProtKB:O00187",
  "gene_name": "Mannan-binding lectin serine protease 2",
  "term_label": "complement activation, lectin pathway"
}